{
  "term_label": "cytoplasm",
  "gene": "UniProtKB:Q86W56",
  "gene_name": "Poly(ADP-ribose) glycohydrolase",
  "gene_symbol": "PARG",
  "term_id": "GO:0005737"
}